{
  "gene_symbol": "GRHL1",
  "gene_name": "Grainyhead-like protein 1 homolog",
  "term_id": "GO:0005634",
  "term_label": "nucleus",
  "gene": "UniProtKB:Q9NZI5"
}